{
  "term_label": "heterochromatin formation",
  "gene_name": "Histone H2A.V",
  "gene_symbol": "H2AZ2",
  "gene": "UniProtKB:Q71UI9",
  "term_id": "GO:0031507"
}